porosome [GO:0033012] (cellular component) Definition: A permanent cup-shaped structure at the cell plasma membrane in secretory cells. Following a secretory stimulus, secretory vesicles transiently dock and fuse at the base of porosomes and release intravesicular contents dictated by the turgor pressure generated from the swelling of secretory vesicles. References: PMID:15090256, PMID:16563225 Relationships: is a type of cellular anatomical structure [GO:0110165]; is part of plasma membrane [GO:0005886]